dendritic cell migration [GO:0036336] (biological process) Subtypes: dendritic cell chemotaxis [GO:0002407] Relationships: is a type of mononuclear cell migration [GO:0071674] Definition: The movement of a dendritic cell within or between different tissues and organs of the body. References: PMID:19339990 Sources: CL:0000451, GOC:nhn